fructose-1-phosphatase activity [GO:0103026] (molecular function) Definition: Catalysis of the reaction: beta-D-fructose 1-phosphate + H2O = D-fructose + phosphate. Relationships: is a type of phosphatase activity [GO:0016791] Sources: RHEA:35603